{
  "term_label": "aggrephagy",
  "gene_name": "Cysteine protease ATG4B",
  "gene": "UniProtKB:Q9Y4P1",
  "term_id": "GO:0035973",
  "gene_symbol": "ATG4B"
}